{
  "term_id": "GO:0008015",
  "gene_symbol": "F5",
  "gene": "UniProtKB:P12259",
  "term_label": "blood circulation",
  "gene_name": "Coagulation factor V"
}